alpha-1D adrenergic receptor binding [GO:0031693] (molecular function) Definition: Binding to an alpha-1D adrenergic receptor. Sources: GOC:mah, GOC:nln Also known as: alpha-1D adrenergic receptor ligand Relationships: is a type of adrenergic receptor binding [GO:0031690]